{
  "term_id": "GO:0005891",
  "term_label": "voltage-gated calcium channel complex",
  "gene": "UniProtKB:O43497",
  "gene_name": "Voltage-dependent T-type calcium channel subunit alpha-1G",
  "gene_symbol": "CACNA1G"
}